N-acetyllactosamine synthase activity [GO:0003945] (molecular function) Relationships: is a type of UDP-galactosyltransferase activity [GO:0035250] Also known as: UDP-galactose:N-acetyl-D-glucosamine 4-beta-D-galactosyltransferase activity, Gal-T, N-acetylglucosamine (beta-1,4)galactosyltransferase activity, N-acetylglucosamine beta-(1,4)-galactosyltransferase activity, N-acetyllactosamine synthetase activity, NAL synthetase activity, UDP-Gal:N-acetylglucosamine beta-1,4-galactosyltransferase activity, UDP-beta-1,4-galactosyltransferase activity, UDP-galactose N-acetylglucosamine beta-4-galactosyltransferase activity, UDP-galactose-N-acetylglucosamine beta-1,4-galactosyltransferase activity, UDP-galactose-N-acetylglucosamine beta-D-galactosyltransferase activity, UDP-galactose-N-acetylglucosamine galactosyltransferase activity, UDP-galactose-acetylglucosamine galactosyltransferase activity, UDP-galactose:N-acetylglucosaminide beta-1,4-galactosyltransferase activity, UDPgalactose-N-acetylglucosamine beta-D-galactosyltransferase activity, UDPgalactose:N-acetyl-D-glucosamine 4-beta-D-galactosyltransferase activity, UDPgalactose:N-acetylglucosaminyl(beta-1,4)galactosyltransferase activity, acetyllactosamine synthetase activity, beta-(1,4)-galactosyltransferase activity, beta-1,4-GalT, beta-1,4-galactosyltransferase activity, beta-N-acetylglucosaminide beta-1,4-galactosyltransferase activity, lactosamine synthase activity, lactosamine synthetase activity, lactose synthetase A protein, uridine diphosphogalactose-acetylglucosamine galactosyltransferase activity Definition: Catalysis of the reaction: UDP-galactose + N-acetyl-D-glucosamine = UDP + N-acetyllactosamine. Sources: EC:2.4.1.90